{
  "term_label": "carbohydrate binding",
  "gene_symbol": "LGALS13",
  "gene_name": "Galactoside-binding soluble lectin 13",
  "term_id": "GO:0030246",
  "gene": "UniProtKB:Q9UHV8"
}